{
  "term_id": "GO:0031669",
  "gene_name": "Urocortin-2",
  "gene": "UniProtKB:Q96RP3",
  "gene_symbol": "UCN2",
  "term_label": "cellular response to nutrient levels"
}